{
  "term_label": "Unknown cellular component",
  "gene_name": "Zinc finger CCCH-type antiviral protein 1-like",
  "gene": "UniProtKB:Q96H79",
  "gene_symbol": "ZC3HAV1L",
  "term_id": "UNKNOWN:0003"
}